{
  "gene_name": "BEN domain-containing protein 3",
  "term_label": "Unknown cellular component",
  "gene": "UniProtKB:Q5T5X7",
  "gene_symbol": "BEND3",
  "term_id": "UNKNOWN:0003"
}